{
  "gene_symbol": "WDR91",
  "gene_name": "WD repeat-containing protein 91",
  "term_id": "GO:0031901",
  "gene": "UniProtKB:A4D1P6",
  "term_label": "early endosome membrane"
}